{
  "gene_name": "Tumor protein p53-inducible nuclear protein 2",
  "gene": "UniProtKB:Q8IXH6",
  "gene_symbol": "TP53INP2",
  "term_id": "GO:0005634",
  "term_label": "nucleus"
}